poly(3-hydroxyalkanoate) binding [GO:0043287] (molecular function) Definition: Binding to a poly(3-hydroxyalkanoate), a polyester of 3-hydroxyacids produced as intracellular granules by a large variety of bacteria. Relationships: is a type of small molecule binding [GO:0036094] Sources: GOC:jl Also known as: PHA binding